{
  "gene": "UniProtKB:Q8N0W5",
  "term_id": "UNKNOWN:0001",
  "gene_name": "IQ domain-containing protein K",
  "gene_symbol": "IQCK",
  "term_label": "Unknown molecular function"
}